regulation of cell growth involved in cardiac muscle cell development [GO:0061050] (biological process) Sources: GOC:dph Relationships: is a type of regulation of cell growth [GO:0001558]; is a type of regulation of cardiac muscle tissue growth [GO:0055021]; regulates GO:0061049 Subtypes: positive regulation of cell growth involved in cardiac muscle cell development [GO:0061051], negative regulation of cell growth involved in cardiac muscle cell development [GO:0061052] Definition: Any process that modulates the rate, frequency, or extent of the growth of a cardiac muscle cell, where growth contributes to the progression of the cell over time from its initial formation to its mature state.